{
  "term_label": "signal transduction",
  "term_id": "GO:0007165",
  "gene": "UniProtKB:Q63HQ2",
  "gene_name": "Pikachurin",
  "gene_symbol": "EGFLAM"
}